chloride transmembrane transport [GO:1902476] (biological process) Relationships: is a type of chloride transport [GO:0006821]; is a type of monoatomic anion transmembrane transport [GO:0098656] Definition: The process in which chloride is transported across a membrane. Sources: GOC:TermGenie, GOC:vw